{
  "gene_name": "Hemicentin-1",
  "term_id": "GO:0098631",
  "gene_symbol": "HMCN1",
  "term_label": "cell adhesion mediator activity",
  "gene": "UniProtKB:Q96RW7"
}